type 7 serotonin receptor binding [GO:0031833] (molecular function) Also known as: 5-hydroxytryptamine 7 receptor binding, type 7 serotonin receptor ligand Sources: GOC:mah, GOC:nln Relationships: is a type of G protein-coupled serotonin receptor binding [GO:0031821] Definition: Binding to a type 7 serotonin receptor.